{
  "term_id": "GO:0005737",
  "gene_symbol": "ALDH3A1",
  "gene_name": "Aldehyde dehydrogenase, dimeric NADP-preferring",
  "term_label": "cytoplasm",
  "gene": "UniProtKB:P30838"
}